vitamin transport [GO:0051180] (biological process) Relationships: is a type of transport [GO:0006810] Also known as: vitamin or cofactor transport Definition: The directed movement of vitamins into, out of or within a cell, or between cells, by means of some agent such as a transporter or pore. A vitamin is one of a number of unrelated organic substances that occur in many foods in small amounts and that are necessary in trace amounts for the normal metabolic functioning of the body. Sources: GOC:ai Subtypes: biotin transport [GO:0015878], GO:0015884, thiamine transport [GO:0015888], GO:0015889, vitamin B6 transport [GO:0031919], riboflavin transport [GO:0032218], vitamin transmembrane transport [GO:0035461], dehydroascorbic acid transport [GO:0070837], GO:0071938